{
  "gene": "UniProtKB:Q86U38",
  "term_id": "GO:0030688",
  "term_label": "preribosome, small subunit precursor",
  "gene_name": "Nucleolar protein 9",
  "gene_symbol": "NOP9"
}